positive regulation of activation-induced cell death of T cells [GO:0070237] (biological process) Also known as: positive regulation of AICD, positive regulation of activated T cell apoptosis, positive regulation of antigen-driven apoptosis, positive regulation of activation-induced cell death of T lymphocytes, positive regulation of activation-induced cell death of T-cells, positive regulation of activation-induced cell death of T-lymphocytes, up regulation of activation-induced cell death of T cells, up-regulation of activation-induced cell death of T cells, upregulation of activation-induced cell death of T cells, activation of activation-induced cell death of T cells, stimulation of activation-induced cell death of T cells Relationships: is a type of positive regulation of immune system process [GO:0002684]; is a type of positive regulation of T cell apoptotic process [GO:0070234]; is a type of GO:0070235; positively regulates activation-induced cell death of T cells [GO:0006924] Sources: GOC:add, ISBN:0781765196 Definition: Any process that activates or increases the frequency, rate or extent of activation-induced cell death of T cells.